{
  "term_id": "UNKNOWN:0001",
  "gene_name": "Cyclin-dependent kinase 2-interacting protein",
  "term_label": "Unknown molecular function",
  "gene_symbol": "CINP",
  "gene": "UniProtKB:Q9BW66"
}